{
  "gene_symbol": "GAB1",
  "gene_name": "GRB2-associated-binding protein 1",
  "gene": "UniProtKB:Q13480",
  "term_id": "GO:0035591",
  "term_label": "signaling adaptor activity"
}